{
  "gene_symbol": "BMP2",
  "term_id": "GO:0001649",
  "gene": "UniProtKB:P12643",
  "gene_name": "Bone morphogenetic protein 2",
  "term_label": "osteoblast differentiation"
}